{
  "term_id": "GO:0005789",
  "gene_name": "Stearoyl-CoA desaturase",
  "gene_symbol": "SCD",
  "gene": "UniProtKB:O00767",
  "term_label": "endoplasmic reticulum membrane"
}